{
  "term_id": "GO:0005634",
  "term_label": "nucleus",
  "gene_symbol": "ALKBH6",
  "gene": "UniProtKB:Q3KRA9",
  "gene_name": "Alpha-ketoglutarate-dependent dioxygenase alkB homolog 6"
}